{
  "term_id": "GO:0043195",
  "gene_name": "Secretagogin",
  "gene": "UniProtKB:O76038",
  "term_label": "terminal bouton",
  "gene_symbol": "SCGN"
}